{
  "gene_name": "Protein phosphatase 1 regulatory subunit 3G",
  "gene_symbol": "PPP1R3G",
  "term_id": "GO:0005979",
  "gene": "UniProtKB:B7ZBB8",
  "term_label": "regulation of glycogen biosynthetic process"
}